regulation of mesenchymal cell proliferation involved in prostate gland development [GO:0060782] (biological process) References: PMID:12221011 Sources: GOC:dph Definition: Any process that modulates the frequency, rate or extent of mesenchymal cell proliferation that contributes to the progression of the prostate gland over time. A mesenchymal cell is a cell that normally gives rise to other cells that are organized as three-dimensional masses, rather than sheets. Relationships: is a type of regulation of mesenchymal cell proliferation [GO:0010464]; regulates mesenchymal cell proliferation involved in prostate gland development [GO:0060781]